embryonic genitalia morphogenesis [GO:0030538] (biological process) Relationships: is a type of GO:0035112; is a type of embryonic organ morphogenesis [GO:0048562] Definition: The process, occurring in the embryo, by which the anatomical structures of the genitalia are generated and organized. Sources: GOC:bf Also known as: embryonic genital morphogenesis